{
  "gene_symbol": "CACNG8",
  "term_label": "AMPA glutamate receptor complex",
  "gene_name": "Voltage-dependent calcium channel gamma-8 subunit",
  "gene": "UniProtKB:Q8WXS5",
  "term_id": "GO:0032281"
}